{
  "term_id": "UNKNOWN:0001",
  "gene_name": "Target of Nesh-SH3",
  "gene": "UniProtKB:Q7Z7G0",
  "term_label": "Unknown molecular function",
  "gene_symbol": "ABI3BP"
}